{
  "term_id": "GO:0004143",
  "gene_name": "Diacylglycerol kinase alpha",
  "term_label": "ATP-dependent diacylglycerol kinase activity",
  "gene": "UniProtKB:P23743",
  "gene_symbol": "DGKA"
}